regulation of zinc ion transmembrane import [GO:0071581] (biological process) Definition: Any process that modulates the frequency, rate or extent of zinc ion import. Relationships: is a type of regulation of zinc ion transmembrane transport [GO:0071580]; regulates zinc ion import across plasma membrane [GO:0071578] Sources: GOC:BHF, GOC:mah Subtypes: negative regulation of zinc ion transmembrane import [GO:0071584]